{
  "gene_symbol": "B4GALNT1",
  "gene": "UniProtKB:Q00973",
  "gene_name": "Beta-1,4 N-acetylgalactosaminyltransferase 1",
  "term_id": "UNKNOWN:0003",
  "term_label": "Unknown cellular component"
}